glycosyltransferase activity [GO:0016757] (molecular function) Sources: GOC:jl, ISBN:0198506732 Also known as: transferase activity, transferring glycosyl groups, transglycosidase activity, transglycosylase activity, transferase activity, transferring other glycosyl groups Relationships: is a type of transferase activity [GO:0016740] Definition: Catalysis of the transfer of a glycosyl group from one compound (donor) to another (acceptor). Subtypes: UDP-glycosyltransferase activity [GO:0008194], sialyltransferase activity [GO:0008373], O-antigen ligase activity [GO:0008754], GO:0008920, GO:0008961, hexosyltransferase activity [GO:0016758], pentosyltransferase activity [GO:0016763], Kdo transferase activity [GO:0043842], S-adenosylmethionine:tRNA ribosyltransferase-isomerase activity [GO:0051075]